protein localization to M-band [GO:0036309] (biological process) Definition: Any process in which a protein is transported to, and/or maintained in, the M band. The M band is the midline of aligned thick filaments in a sarcomere. References: PMID:18782775 Sources: GOC:BHF, GOC:rl Relationships: is a type of protein localization to organelle [GO:0033365] Also known as: cellular protein localization to M-band, protein localization to M disc, protein localization to mesophragma, protein localization to M line